anandamide 11,12 epoxidase activity [GO:0062188] (molecular function) References: PMID:21289075 Sources: RHEA:53144 Definition: Catalysis of the reaction: N-(5Z,8Z,11Z,14Z-eicosatetraenoyl)-ethanolamine + O2 + reduced [NADPH--hemoprotein reductase] = H+ + H2O + N-(11,12-epoxy-5Z,8Z,14Z-eicosatrienoyl)-ethanolamine + oxidized [NADPH--hemoprotein reductase]. Relationships: is_a anandamide epoxidase activity [GO:0062186]